{
  "term_id": "GO:0045824",
  "gene_name": "NLR family CARD domain-containing protein 3",
  "gene": "UniProtKB:Q7RTR2",
  "gene_symbol": "NLRC3",
  "term_label": "negative regulation of innate immune response"
}